negative regulation of collagen fibril organization [GO:1904027] (biological process) Definition: Any process that stops, prevents or reduces the frequency, rate or extent of collagen fibril organization. References: PMID:25451920 Sources: GOC:TermGenie, GO_REF:0000058 Relationships: is a type of negative regulation of extracellular matrix organization [GO:1903054]; is a type of GO:1904026; negatively regulates GO:0030199 Also known as: down regulation of collagen fibril organisation, down regulation of collagen fibril organization, down regulation of fibrillar collagen organization, down-regulation of collagen fibril organisation, down-regulation of collagen fibril organization, down-regulation of fibrillar collagen organization, downregulation of collagen fibril organisation, downregulation of collagen fibril organization, downregulation of fibrillar collagen organization, negative regulation of collagen fibril organisation, negative regulation of fibrillar collagen organization, inhibition of collagen fibril organisation, inhibition of collagen fibril organization, inhibition of fibrillar collagen organization